{
  "gene_symbol": "C18orf63",
  "gene": "UniProtKB:Q68DL7",
  "term_id": "UNKNOWN:0001",
  "term_label": "Unknown molecular function",
  "gene_name": "Uncharacterized protein C18orf63"
}